Grb2-Shc complex [GO:0070437] (cellular component) Relationships: is a type of plasma membrane protein complex [GO:0098797] Also known as: Grb2-Shc complex, EGF stimulated References: PMID:7798267 Sources: GOC:mah Definition: A protein complex that contains Grb2 and the adaptor protein Shc, and is involved in linking epidermal growth factor receptor (EGFR) activation to the p21-Ras pathway.